{
  "gene_symbol": "ABHD15",
  "gene_name": "Protein ABHD15",
  "term_label": "Unknown cellular component",
  "term_id": "UNKNOWN:0003",
  "gene": "UniProtKB:Q6UXT9"
}